{
  "gene_name": "Putative serine protease 29",
  "term_label": "proteolysis",
  "gene": "UniProtKB:A6NIE9",
  "gene_symbol": "PRSS29P",
  "term_id": "GO:0006508"
}